glutathione S-conjugate carboxypeptidase activity [GO:0102274] (MF) Definition: Catalysis of the reaction: an S-substituted glutathione + H2O = glycine + S-substituted gamma-glutamyl-L-cysteine. Patricipates in glutathione-mediated detoxification. Sources: RHEA:60448 Relationships: is_a metallocarboxypeptidase activity [GO:0004181]